negative regulation of kidney development [GO:0090185] (biological process) Also known as: negative regulation of nephrogenesis Relationships: is a type of GO:0051093; is_a negative regulation of multicellular organismal process [GO:0051241]; is a type of regulation of kidney development [GO:0090183]; negatively regulates kidney development [GO:0001822] Sources: GOC:dph, GOC:tb, GOC:yaf Subtypes: negative regulation of mesonephros development [GO:0061218], negative regulation of nephron tubule epithelial cell differentiation [GO:0072183], GO:0072217, GO:0090194 Definition: Any process that decreases the rate, frequency or extent of kidney development. Kidney development is the process whose specific outcome is the progression of the kidney over time, from its formation to the mature structure. The kidney is an organ that filters the blood and excretes the end products of body metabolism in the form of urine.